{
  "gene_symbol": "HSP90AB3P",
  "gene_name": "Putative heat shock protein HSP 90-beta-3",
  "term_id": "GO:0016887",
  "gene": "UniProtKB:Q58FF7",
  "term_label": "ATP hydrolysis activity"
}